{
  "gene_symbol": "RPL41",
  "term_id": "GO:0022625",
  "gene": "UniProtKB:P62945",
  "term_label": "cytosolic large ribosomal subunit",
  "gene_name": "Large ribosomal subunit protein eL41"
}